response to fungus [GO:0009620] (biological process) Sources: GOC:hb Also known as: response to fungi Subtypes: GO:0001878, response to symbiotic fungus [GO:0009610], detection of fungus [GO:0016046], defense response to fungus [GO:0050832] Relationships: is a type of response to other organism [GO:0051707] Definition: Any process that results in a change in state or activity of a cell or an organism (in terms of movement, secretion, enzyme production, gene expression, etc.) as a result of a stimulus from a fungus.